{
  "gene_name": "Cyclin-dependent kinase 12",
  "gene": "UniProtKB:Q9NYV4",
  "term_label": "RNA polymerase II CTD heptapeptide repeat kinase activity",
  "term_id": "GO:0008353",
  "gene_symbol": "CDK12"
}